{
  "term_label": "Unknown biological process",
  "gene": "UniProtKB:Q8IZP2",
  "gene_name": "Putative protein FAM10A4",
  "term_id": "UNKNOWN:0002",
  "gene_symbol": "ST13P4"
}